{
  "term_label": "Unknown biological process",
  "gene_name": "Glutamine and serine-rich protein 1",
  "gene": "UniProtKB:Q2KHR3",
  "term_id": "UNKNOWN:0002",
  "gene_symbol": "QSER1"
}